{
  "term_label": "ATF4-CREB1 transcription factor complex",
  "gene_symbol": "CREM",
  "gene": "UniProtKB:Q03060",
  "gene_name": "cAMP-responsive element modulator",
  "term_id": "GO:1990589"
}